{
  "gene_symbol": "HPR",
  "gene_name": "Haptoglobin-related protein",
  "gene": "UniProtKB:P00739",
  "term_label": "blood microparticle",
  "term_id": "GO:0072562"
}